{
  "gene": "UniProtKB:A1Z1Q3",
  "gene_symbol": "MACROD2",
  "term_id": "GO:0140293",
  "term_label": "ADP-ribosylglutamate hydrolase activity",
  "gene_name": "ADP-ribose glycohydrolase MACROD2"
}